{
  "gene_name": "Transcription factor 7-like 2",
  "term_label": "beta-catenin-TCF complex",
  "gene_symbol": "TCF7L2",
  "gene": "UniProtKB:Q9NQB0",
  "term_id": "GO:1990907"
}